investment cone [GO:0070865] (cellular component) Definition: A cytoskeletal part that consists of a microfilament-rich cone that forms round each nucleus in a spermatogenic cyst and translocates the length of the cyst during sperm individualization. References: PMID:15829565, PMID:9550716 Sources: GOC:sart Relationships: is a type of cellular anatomical structure [GO:0110165]; is part of cytoskeleton [GO:0005856]; is part of sperm individualization complex [GO:0070864] Also known as: F-actin cone